{
  "gene_symbol": "ARHGEF9",
  "gene": "UniProtKB:O43307",
  "term_id": "GO:0099150",
  "gene_name": "Rho guanine nucleotide exchange factor 9",
  "term_label": "regulation of postsynaptic specialization assembly"
}